short tract gene conversion [GO:0035823] (biological process) References: PMID:16954385 Sources: GOC:mah Definition: A gene conversion process in which a segment of about 50-200 base pairs is transferred from the donor to the acceptor. Relationships: is a type of gene conversion [GO:0035822]